{
  "gene_name": "Leucine-rich repeat transmembrane neuronal protein 1",
  "gene": "UniProtKB:Q86UE6",
  "term_id": "GO:0038023",
  "term_label": "signaling receptor activity",
  "gene_symbol": "LRRTM1"
}